{
  "gene_name": "DNA-directed RNA polymerase II subunit RPB2",
  "term_id": "GO:0006367",
  "gene_symbol": "POLR2B",
  "term_label": "transcription initiation at RNA polymerase II promoter",
  "gene": "UniProtKB:P30876"
}